{
  "gene": "UniProtKB:Q96KN7",
  "gene_symbol": "RPGRIP1",
  "term_label": "Unknown molecular function",
  "term_id": "UNKNOWN:0001",
  "gene_name": "X-linked retinitis pigmentosa GTPase regulator-interacting protein 1"
}